{
  "gene_symbol": "FGF20",
  "term_label": "neurogenesis",
  "gene_name": "Fibroblast growth factor 20",
  "gene": "UniProtKB:Q9NP95",
  "term_id": "GO:0022008"
}